{
  "term_label": "plasma membrane",
  "term_id": "GO:0005886",
  "gene": "UniProtKB:P36888",
  "gene_symbol": "FLT3",
  "gene_name": "Receptor-type tyrosine-protein kinase FLT3"
}